{
  "gene": "UniProtKB:B8ZZ34",
  "term_id": "GO:0048172",
  "gene_symbol": "SHISA8",
  "gene_name": "Protein shisa-8",
  "term_label": "regulation of short-term neuronal synaptic plasticity"
}